{
  "term_id": "GO:0005739",
  "gene_name": "Hydroxymethylglutaryl-CoA lyase, mitochondrial",
  "gene_symbol": "HMGCL",
  "gene": "UniProtKB:P35914",
  "term_label": "mitochondrion"
}